{
  "gene_symbol": "STAC3",
  "gene": "UniProtKB:Q96MF2",
  "term_id": "UNKNOWN:0001",
  "gene_name": "SH3 and cysteine-rich domain-containing protein 3",
  "term_label": "Unknown molecular function"
}